{
  "term_id": "UNKNOWN:0002",
  "term_label": "Unknown biological process",
  "gene": "UniProtKB:Q9BSA4",
  "gene_symbol": "TTYH2",
  "gene_name": "Protein tweety homolog 2"
}